{
  "term_id": "GO:0005886",
  "gene": "UniProtKB:O95484",
  "gene_name": "Claudin-9",
  "gene_symbol": "CLDN9",
  "term_label": "plasma membrane"
}